{
  "term_label": "U5 snRNP",
  "gene_name": "Small nuclear ribonucleoprotein Sm D2",
  "gene_symbol": "SNRPD2",
  "term_id": "GO:0005682",
  "gene": "UniProtKB:P62316"
}